{
  "gene": "UniProtKB:Q8N6V9",
  "gene_name": "Testis-expressed protein 9",
  "gene_symbol": "TEX9",
  "term_label": "Unknown molecular function",
  "term_id": "UNKNOWN:0001"
}